{
  "gene_symbol": "PDX1",
  "term_id": "GO:0003309",
  "term_label": "type B pancreatic cell differentiation",
  "gene_name": "Pancreas_duodenum homeobox protein 1",
  "gene": "UniProtKB:P52945"
}